{
  "term_id": "GO:0019773",
  "gene_symbol": "PSMA3",
  "gene_name": "Proteasome subunit alpha type-3",
  "term_label": "proteasome core complex, alpha-subunit complex",
  "gene": "UniProtKB:P25788"
}